{
  "term_id": "GO:0070106",
  "gene_name": "2'-5'-oligoadenylate synthase 3",
  "gene": "UniProtKB:Q9Y6K5",
  "term_label": "interleukin-27-mediated signaling pathway",
  "gene_symbol": "OAS3"
}